CHOP-ATF4 complex [GO:1990617] (cellular component) Also known as: ATF4-CHOP heterodimer, CHOP-ATF4 heterodimer, CHOP-CREB-2 complex, CHOP/ATF4 complex, GADD153-ATF4 complex Definition: A heterodimeric transcription factor complex that is composed of CHOP (C/EBP homology protein, GADD153) and ATF4 (activating transcription factor 4, also known as cAMP response element binding protein-2/CREB-2) subunits. References: PMID:18940792 Sources: GOC:PARL, GOC:bf Relationships: is a type of RNA polymerase II transcription regulator complex [GO:0090575]